{
  "gene": "UniProtKB:Q8IXA5",
  "gene_name": "Sperm acrosome membrane-associated protein 3",
  "term_label": "fusion of sperm to egg plasma membrane involved in single fertilization",
  "term_id": "GO:0007342",
  "gene_symbol": "SPACA3"
}